{
  "term_label": "RNA binding",
  "gene": "UniProtKB:Q9H171",
  "gene_symbol": "ZBP1",
  "gene_name": "Z-DNA-binding protein 1",
  "term_id": "GO:0003723"
}